{
  "term_id": "GO:0004252",
  "gene_symbol": "GZMM",
  "gene": "UniProtKB:P51124",
  "term_label": "serine-type endopeptidase activity",
  "gene_name": "Granzyme M"
}